{
  "gene_symbol": "LRPAP1",
  "gene": "UniProtKB:P30533",
  "term_label": "low-density lipoprotein particle receptor binding",
  "gene_name": "Alpha-2-macroglobulin receptor-associated protein",
  "term_id": "GO:0050750"
}